{
  "gene_symbol": "C1QTNF1",
  "term_id": "GO:0005615",
  "gene_name": "Complement C1q tumor necrosis factor-related protein 1",
  "term_label": "extracellular space",
  "gene": "UniProtKB:Q9BXJ1"
}